hepatoblast apoptotic process [GO:1902489] (biological process) Relationships: is a type of apoptotic process [GO:0006915] Definition: Any apoptotic process in a hepatoblast. Also known as: hepatoblast apoptosis References: PMID:22412967 Sources: GOC:TermGenie